lateral sprouting involved in mammary gland duct morphogenesis [GO:0060599] (biological process) Also known as: mammary gland duct secondary branching References: PMID:17120154 Sources: GOC:dph Definition: The process in which a branch forms along the side of a mammary duct. Relationships: is a type of lateral sprouting from an epithelium [GO:0060601]; BFO_0000050 branching involved in mammary gland duct morphogenesis [GO:0060444]